{
  "gene_symbol": "TRBV7-7",
  "term_id": "GO:0005886",
  "term_label": "plasma membrane",
  "gene": "UniProtKB:A0A0K0K1E9",
  "gene_name": "T cell receptor beta variable 7-7"
}